{
  "gene": "UniProtKB:Q86WW8",
  "term_label": "Unknown molecular function",
  "gene_name": "Cytochrome c oxidase assembly factor 5",
  "term_id": "UNKNOWN:0001",
  "gene_symbol": "COA5"
}